{
  "gene": "UniProtKB:P62324",
  "term_label": "negative regulation of cell population proliferation",
  "gene_symbol": "BTG1",
  "term_id": "GO:0008285",
  "gene_name": "Protein BTG1"
}